histidinol dehydrogenase activity [GO:0004399] (molecular function) Relationships: is_a oxidoreductase activity, acting on the CH-OH group of donors, NAD or NADP as acceptor [GO:0016616] Definition: Catalysis of the reaction: H2O + L-histidinol + 2 NAD+ = 3 H+ + L-histidine + 2 NADH. Sources: RHEA:20641